CGRP receptor complex [GO:1990406] (cellular component) Definition: A transmembrane, G protein-coupled signaling receptor complex recognized by calcitonin gene-related peptides (CGRP). References: PMID:20826335 Sources: GOC:bhm Also known as: CGRP-R complex, Calcitonin-gene-related peptide receptor complex, calcitonin gene-related polypeptide receptor complex Note: An example of this is CALCRL in human (Q16602) in PMID:20826335 (inferred from direct assay). Relationships: is a type of calcitonin family receptor complex [GO:1903439]